{
  "term_id": "UNKNOWN:0001",
  "gene_name": "Probable non-functional immunoglobulin lambda variable 2-33",
  "term_label": "Unknown molecular function",
  "gene_symbol": "IGLV2-33",
  "gene": "UniProtKB:A0A075B6J2"
}